{
  "term_id": "GO:0036503",
  "gene_name": "UBX domain-containing protein 4",
  "gene": "UniProtKB:Q92575",
  "gene_symbol": "UBXN4",
  "term_label": "ERAD pathway"
}